{
  "gene": "UniProtKB:Q14135",
  "gene_symbol": "VGLL4",
  "gene_name": "Transcription cofactor vestigial-like protein 4",
  "term_id": "GO:0001223",
  "term_label": "transcription coactivator binding"
}